{
  "gene_symbol": "ADAM2",
  "gene_name": "Disintegrin and metalloproteinase domain-containing protein 2",
  "gene": "UniProtKB:Q99965",
  "term_id": "GO:0006508",
  "term_label": "proteolysis"
}